{
  "term_id": "GO:0004674",
  "term_label": "protein serine/threonine kinase activity",
  "gene": "UniProtKB:P54646",
  "gene_symbol": "PRKAA2",
  "gene_name": "5'-AMP-activated protein kinase catalytic subunit alpha-2"
}